{
  "gene_symbol": "JPT2",
  "gene": "UniProtKB:Q9H910",
  "term_id": "UNKNOWN:0001",
  "term_label": "Unknown molecular function",
  "gene_name": "Jupiter microtubule associated homolog 2"
}